{
  "gene_name": "Coiled-coil domain-containing protein 40",
  "gene": "UniProtKB:Q4G0X9",
  "term_label": "epithelial cilium movement involved in determination of left/right asymmetry",
  "term_id": "GO:0060287",
  "gene_symbol": "CCDC40"
}